{
  "term_label": "cytokine-mediated signaling pathway",
  "term_id": "GO:0019221",
  "gene_name": "Tissue factor",
  "gene": "UniProtKB:P13726",
  "gene_symbol": "F3"
}